{
  "gene": "UniProtKB:O60504",
  "term_id": "GO:0005886",
  "gene_name": "Vinexin",
  "term_label": "plasma membrane",
  "gene_symbol": "SORBS3"
}